postsynaptic endocytic zone [GO:0098843] (cellular component) Relationships: is a type of cellular anatomical structure [GO:0110165]; is part of GO:0098794; has part clathrin coat [GO:0030118] References: PMID:17880892 Definition: A stably positioned site of clathrin adjacent and physically attached to the postsynaptic specialization, which is the site of endocytosis of post-synaptic proteins.